urea:sodium symporter activity [GO:0015401] (molecular function) Sources: TC:2.A.21.6.1 Also known as: urea active transmembrane transporter activity Relationships: is a type of GO:0015204; is_a GO:0015370 Definition: Enables the transfer of a solute or solutes from one side of a membrane to the other according to the reaction: urea(out) + Na+(out) = urea(in) + Na+(in).